plastid inner membrane organization [GO:0009667] (biological process) Sources: GOC:ai, GOC:dph, GOC:jl, GOC:mah Definition: A process that is carried out at the cellular level which results in the assembly, arrangement of constituent parts, or disassembly of the inner membrane of a plastid. Also known as: plastid inner membrane organisation, plastid inner membrane organization and biogenesis Relationships: is a type of GO:0009668